{
  "gene": "UniProtKB:A0A0B4J240",
  "term_id": "GO:0009617",
  "gene_name": "T cell receptor alpha variable 10",
  "gene_symbol": "TRAV10",
  "term_label": "response to bacterium"
}